{
  "term_label": "protein kinase activator activity",
  "gene_name": "Large ribosomal subunit protein P1",
  "gene_symbol": "RPLP1",
  "term_id": "GO:0030295",
  "gene": "UniProtKB:P05386"
}